uracil salvage [GO:0006223] (biological process) Relationships: is a type of pyrimidine nucleobase salvage [GO:0043100]; is a type of uracil biosynthetic process [GO:0046107] Definition: Any process that generates uracil, 2,4-dioxopyrimidine, from derivatives of it without de novo synthesis. Sources: GOC:jl